{
  "gene": "UniProtKB:O60921",
  "term_label": "mitotic intra-S DNA damage checkpoint signaling",
  "gene_name": "Checkpoint protein HUS1",
  "gene_symbol": "HUS1",
  "term_id": "GO:0031573"
}